{
  "gene_name": "UDP-glucuronosyltransferase 1-6",
  "term_label": "cellular response to glucocorticoid stimulus",
  "term_id": "GO:0071385",
  "gene_symbol": "UGT1A6",
  "gene": "UniProtKB:P19224"
}